{
  "gene_name": "Enhancer of mRNA-decapping protein 3",
  "gene_symbol": "EDC3",
  "term_label": "P-body",
  "term_id": "GO:0000932",
  "gene": "UniProtKB:Q96F86"
}